{
  "gene_symbol": "USP17L30",
  "term_id": "GO:0004843",
  "gene": "UniProtKB:Q0WX57",
  "gene_name": "Ubiquitin carboxyl-terminal hydrolase 17-like protein 24",
  "term_label": "cysteine-type deubiquitinase activity"
}